{
  "gene_symbol": "MTFR2",
  "gene_name": "Mitochondrial fission regulator 2",
  "term_label": "mitochondrial fission",
  "gene": "UniProtKB:Q6P444",
  "term_id": "GO:0000266"
}